{
  "term_id": "GO:0005912",
  "gene": "UniProtKB:O00151",
  "term_label": "adherens junction",
  "gene_name": "PDZ and LIM domain protein 1",
  "gene_symbol": "PDLIM1"
}